{
  "gene_name": "Rho GDP-dissociation inhibitor 3",
  "gene": "UniProtKB:Q99819",
  "gene_symbol": "ARHGDIG",
  "term_id": "GO:0005829",
  "term_label": "cytosol"
}